6'-deoxychalcone synthase activity [GO:0033808] (molecular function) Relationships: is a type of GO:0016747 Sources: EC:2.3.1.170 Also known as: malonyl-CoA:4-coumaroyl-CoA malonyltransferase (cyclizing, reducing) activity Definition: Catalysis of the reaction: 3 malonyl-CoA + 4-coumaroyl-CoA + NADPH + H+ = 4 CoA + isoliquiritigenin + 3 CO2 + NADP+ + H2O.